response to aldosterone [GO:1904044] (biological process) Definition: Any process that results in a change in state or activity of a cell or an organism (in terms of movement, secretion, enzyme production, gene expression, etc.) as a result of an aldosterone stimulus. References: PMID:17644563 Sources: GOC:TermGenie, GO_REF:0000071 Relationships: is a type of response to mineralocorticoid [GO:0051385]; is a type of response to alcohol [GO:0097305]; is a type of response to ketone [GO:1901654] Subtypes: GO:1904045